{
  "term_label": "small ribosomal subunit",
  "gene": "UniProtKB:P62269",
  "gene_name": "Small ribosomal subunit protein uS13",
  "term_id": "GO:0015935",
  "gene_symbol": "RPS18"
}